{
  "term_id": "UNKNOWN:0001",
  "gene": "UniProtKB:Q9Y394",
  "gene_symbol": "DHRS7",
  "gene_name": "Dehydrogenase_reductase SDR family member 7",
  "term_label": "Unknown molecular function"
}